positive regulation of shoot apical meristem development [GO:1902185] (biological process) References: PMID:21496644 Sources: GOC:TermGenie Relationships: is a type of positive regulation of developmental process [GO:0051094]; is a type of regulation of shoot apical meristem development [GO:1902183]; positively regulates shoot apical meristem development [GO:1902182] Also known as: activation of promeristem development, positive regulation of promeristem development, up regulation of promeristem development, up-regulation of promeristem development, upregulation of promeristem development, activation of SAM development, positive regulation of SAM development, up regulation of SAM development, up regulation of shoot apical meristem development, up-regulation of SAM development, up-regulation of shoot apical meristem development, upregulation of SAM development, upregulation of shoot apical meristem development, activation of shoot apical meristem development, activation of primary shoot meristem development, positive regulation of primary shoot meristem development, up regulation of primary shoot meristem development, up-regulation of primary shoot meristem development, upregulation of primary shoot meristem development Definition: Any process that activates or increases the frequency, rate or extent of shoot apical meristem development.